ureteric bud invasion [GO:0072092] (biological process) Sources: GOC:mtg_kidney_jan10 Definition: The process in which the ureteric bud grows along its axis and contributes to the formation of the metanephros. Relationships: is_a developmental growth involved in morphogenesis [GO:0060560]; is part of GO:0060677; is part of metanephric renal vesicle formation [GO:0072093]